{
  "term_label": "Unknown cellular component",
  "gene_name": "Intermembrane lipid transfer protein VPS13C",
  "gene": "UniProtKB:Q709C8",
  "gene_symbol": "VPS13C",
  "term_id": "UNKNOWN:0003"
}